{
  "gene_symbol": "FKBP10",
  "gene": "UniProtKB:Q96AY3",
  "term_label": "protein folding",
  "term_id": "GO:0006457",
  "gene_name": "Peptidyl-prolyl cis-trans isomerase FKBP10"
}